netrin receptor activity involved in chemorepulsion [GO:0005043] (MF) Definition: Combining with a netrin signal and transmitting the signal from one side of the membrane to the other to contribute to the directed movement of a motile cell away from a higher concentration of netrin. Relationships: is_a GO:0005042; is part of negative chemotaxis [GO:0050919] Also known as: netrin receptor activity involved in negative chemotaxis, repulsive netrin receptor activity Sources: GOC:dph, GOC:signaling